phenylacetate catabolic process [GO:0010124] (biological process) Sources: GOC:pz Relationships: is a type of GO:0042178; is a type of benzene-containing compound metabolic process [GO:0042537]; is a type of monocarboxylic acid catabolic process [GO:0072329] Definition: The chemical reactions and pathways resulting in the breakdown of phenylacetate. Also known as: phenylacetate breakdown, phenylacetate catabolism, phenylacetate degradation